BMP receptor activity [GO:0098821] (molecular function) Definition: Combining with a member of the bone morphogenetic protein (BMP) family, and transmitting a signal across the plasma membrane to initiate a change in cell activity. Relationships: is a type of GO:0004675; is part of GO:0030509 Sources: GOC:BHF, GOC:dos